{
  "term_label": "Unknown molecular function",
  "gene": "UniProtKB:Q9UGC7",
  "gene_name": "Peptide chain release factor 1-like, mitochondrial",
  "gene_symbol": "MTRF1L",
  "term_id": "UNKNOWN:0001"
}